{
  "term_id": "UNKNOWN:0001",
  "gene": "UniProtKB:Q5VZI3",
  "gene_symbol": "TMEM268",
  "gene_name": "Transmembrane protein 268",
  "term_label": "Unknown molecular function"
}